{
  "term_label": "mitotic chromosome condensation",
  "gene_symbol": "NCAPH",
  "term_id": "GO:0007076",
  "gene": "UniProtKB:Q15003",
  "gene_name": "Condensin complex subunit 2"
}